{
  "gene_symbol": "SORBS1",
  "gene_name": "Sorbin and SH3 domain-containing protein 1",
  "term_id": "GO:0005737",
  "term_label": "cytoplasm",
  "gene": "UniProtKB:Q9BX66"
}